Notch signaling pathway involved in negative regulation of venous endothelial cell fate commitment [GO:2000796] (biological process) Definition: Any Notch signaling pathway that is involved in negative regulation of venous endothelial cell fate commitment. References: PMID:11585794 Also known as: N signaling pathway involved in negative regulation of venous endothelial cell fate commitment, Notch receptor signaling pathway involved in negative regulation of venous endothelial cell fate commitment, Notch receptor signalling pathway involved in negative regulation of venous endothelial cell fate commitment, Notch signalling pathway involved in negative regulation of venous endothelial cell fate commitment, Notch-receptor signaling pathway involved in negative regulation of venous endothelial cell fate commitment, Notch-receptor signalling pathway involved in negative regulation of venous endothelial cell fate commitment Relationships: is a type of GO:0007219; is part of negative regulation of venous endothelial cell fate commitment [GO:2000788]